deoxyhypusine monooxygenase activity [GO:0019135] (MF) Definition: Catalysis of the reaction: protein N6-(4-aminobutyl)-L-lysine + donor-H2 + O2 = protein N6-((R)-4-amino-2-hydroxybutyl)-L-lysine + acceptor + H2O. Also known as: deoxyhypusine hydroxylase activity, DOHH activity, deoxyhypusine dioxygenase activity, deoxyhypusine,hydrogen-donor:oxygen oxidoreductase (2-hydroxylating) Sources: EC:1.14.99.29 Relationships: is_a GO:0004497; is a type of oxidoreductase activity, acting on paired donors, with incorporation or reduction of molecular oxygen [GO:0016705]; is a type of GO:0140096